{
  "term_label": "extracellular region",
  "gene_symbol": "SPINK7",
  "gene_name": "Serine protease inhibitor Kazal-type 7",
  "term_id": "GO:0005576",
  "gene": "UniProtKB:P58062"
}